{
  "gene": "UniProtKB:Q14956",
  "gene_name": "Transmembrane glycoprotein NMB",
  "term_id": "GO:0005886",
  "gene_symbol": "GPNMB",
  "term_label": "plasma membrane"
}